{
  "term_label": "extracellular space",
  "gene_name": "Eotaxin",
  "gene_symbol": "CCL11",
  "term_id": "GO:0005615",
  "gene": "UniProtKB:P51671"
}